mesodermal cell migration [GO:0008078] (biological process) References: PMID:25119047 Sources: GOC:ascb_2009, GOC:dph, GOC:mah, GOC:sat, GOC:tb Relationships: is a type of ameboidal-type cell migration [GO:0001667] Subtypes: mesoderm migration involved in gastrulation [GO:0007509] Definition: The orderly movement of mesodermal cells from one site to another. Also known as: mesoderm cell migration